interleukin-3 receptor complex [GO:0005894] (cellular component) Definition: A protein complex that binds interleukin-3; comprises an alpha and a beta subunit. The alpha chain is specific to the interleukin-3 receptor, whereas the beta chain is shared with the receptors for granulocyte-macrophage colony-stimulating factor and interleukin-5. Also known as: IL-3 receptor complex References: PMID:11839579 Relationships: is a type of plasma membrane signaling receptor complex [GO:0098802]